{
  "term_id": "GO:0006620",
  "gene": "UniProtKB:P11441",
  "gene_name": "Ubiquitin-like protein 4A",
  "gene_symbol": "UBL4A",
  "term_label": "post-translational protein targeting to endoplasmic reticulum membrane"
}